{
  "term_id": "GO:0045087",
  "gene_symbol": "APCS",
  "term_label": "innate immune response",
  "gene_name": "Serum amyloid P-component",
  "gene": "UniProtKB:P02743"
}